{
  "term_label": "transcription elongation factor activity",
  "gene_name": "Transcription elongation factor A N-terminal and central domain-containing protein",
  "gene": "UniProtKB:Q8N8B7",
  "term_id": "GO:0003711",
  "gene_symbol": "TCEANC"
}